{
  "term_label": "extracellular region",
  "gene_name": "Thrombopoietin",
  "gene_symbol": "THPO",
  "term_id": "GO:0005576",
  "gene": "UniProtKB:P40225"
}